{
  "term_id": "GO:0005229",
  "gene_name": "Protein tweety homolog 3",
  "gene": "UniProtKB:Q9C0H2",
  "term_label": "intracellularly calcium-gated chloride channel activity",
  "gene_symbol": "TTYH3"
}